positive regulation of interleukin-35 production [GO:0070756] (biological process) Also known as: positive regulation of IL-35 production, up regulation of interleukin-35 production, up-regulation of interleukin-35 production, upregulation of interleukin-35 production, activation of interleukin-35 production, positive regulation of interleukin-35 biosynthetic process, stimulation of interleukin-35 production Sources: GOC:mah Relationships: is a type of positive regulation of cytokine production [GO:0001819]; is a type of regulation of interleukin-35 production [GO:0070754]; positively regulates interleukin-35 production [GO:0070753] Definition: Any process that activates or increases the frequency, rate, or extent of interleukin-35 production.